{
  "gene_name": "Tetraspanin-8",
  "term_id": "UNKNOWN:0001",
  "gene": "UniProtKB:P19075",
  "term_label": "Unknown molecular function",
  "gene_symbol": "TSPAN8"
}